{
  "gene_name": "DNA-binding protein RFX7",
  "gene_symbol": "RFX7",
  "term_label": "DNA-binding transcription factor activity, RNA polymerase II-specific",
  "gene": "UniProtKB:Q2KHR2",
  "term_id": "GO:0000981"
}